carbohydrate:proton symporter activity [GO:0005351] (molecular function) Relationships: is a type of carbohydrate:monoatomic cation symporter activity [GO:0005402]; is a type of solute:proton symporter activity [GO:0015295] Sources: TC:2.A.1.1 Definition: Enables the transfer of a solute or solutes from one side of a membrane to the other according to the reaction: carbohydrate(out) + H+(out) = carbohydrate(in) + H+(in). Also known as: hydrogen:sugar transporter activity, sugar transporter, proton:sugar symporter activity, sugar:hydrogen symporter activity, cation/sugar symporter activity, hydrogen:sugar symporter activity, lactose/glucose efflux transporter activity, sugar efflux transmembrane transporter activity, sugar porter activity, sugar:hydrogen ion symporter activity, sugar:proton symporter activity Subtypes: GO:0005364, sucrose:proton symporter activity [GO:0008506], hexose:proton symporter activity [GO:0009679], arabinose:proton symporter activity [GO:0015518], D-xylose:proton symporter activity [GO:0015519], lactose:proton symporter activity [GO:0015528], raffinose:proton symporter activity [GO:0015529], 2-keto-3-deoxygluconate:proton symporter activity [GO:0015649], GO:0044693